{
  "gene": "UniProtKB:Q6I9Y2",
  "term_id": "GO:0000445",
  "term_label": "THO complex part of transcription export complex",
  "gene_name": "THO complex subunit 7 homolog",
  "gene_symbol": "THOC7"
}